aldehyde dehydrogenase (NAD+) activity [GO:0004029] (molecular function) Sources: RHEA:16185 Subtypes: retinal dehydrogenase (NAD+) activity [GO:0001758], GO:0008802, lactaldehyde dehydrogenase (NAD+) activity [GO:0008911], phenylacetaldehyde dehydrogenase (NAD+) activity [GO:0008957], formaldehyde dehydrogenase (NAD+) activity [GO:0018467], 2-formylbenzoate dehydrogenase (NAD+) activity [GO:0018474], benzaldehyde dehydrogenase (NAD+) activity [GO:0018479], GO:0018484, salicylaldehyde dehydrogenase (NAD+) activity [GO:0018485], aryl-aldehyde dehydrogenase (NAD+) activity [GO:0019108], GO:0019145, fluoroacetaldehyde dehydrogenase (NAD+) activity [GO:0033723], abieta-7,13-dien-18-al (NAD+) dehydrogenase activity [GO:0036188], GO:0047106, gamma-guanidinobutyraldehyde dehydrogenase (NAD+) activity [GO:0047107], GO:0047551, glycolaldehyde dehydrogenase (NAD+) activity [GO:0050569], GO:0102244, fatty aldehyde dehydrogenase (NAD+) activity [GO:0102673], GO:0106373, farnesal dehydrogenase (NAD+) activity [GO:0120553], acetaldehyde dehydrogenase (NAD+) activity [GO:0140087] Definition: Catalysis of the reaction: an aldehyde + H2O + NAD+ = a carboxylate + 2 H+ + NADH. Relationships: is_a aldehyde dehydrogenase [NAD(P)+] activity [GO:0004030] Also known as: CoA-independent aldehyde dehydrogenase activity, NAD-aldehyde dehydrogenase activity, NAD-dependent 4-hydroxynonenal dehydrogenase activity, NAD-dependent aldehyde dehydrogenase activity, NAD-linked aldehyde dehydrogenase activity, aldehyde dehydrogenase (NAD+), aldehyde:NAD+ oxidoreductase activity, m-methylbenzaldehyde dehydrogenase activity, propionaldehyde dehydrogenase activity Regulation: negatively regulated by aldehyde dehydrogenase (NAD+) inhibitor activity [GO:0140631]